retina development in camera-type eye [GO:0060041] (biological process) Also known as: retina development in camera-style eye, retinal development Sources: GOC:bf, GOC:dph, ISBN:0815340729 Relationships: is a type of anatomical structure development [GO:0048856]; is part of camera-type eye development [GO:0043010] Definition: The process whose specific outcome is the progression of the retina over time, from its formation to the mature structure. The retina is the innermost layer or coating at the back of the eyeball, which is sensitive to light and in which the optic nerve terminates. Regulation: regulated by regulation of retina development in camera-type eye [GO:1902866]; negatively regulated by negative regulation of retina development in camera-type eye [GO:1902867]; positively regulated by positive regulation of retina development in camera-type eye [GO:1902868]